methotrexate binding [GO:0051870] (molecular function) Definition: Binding to methotrexate, an antineoplastic antimetabolite with immunosuppressant properties. It is an inhibitor of tetrahydrofolate reductase and prevents the formation of tetrahydrofolate, necessary for synthesis of thymidylate, an essential component of DNA. Sources: GOC:nln Relationships: is a type of carboxylic acid binding [GO:0031406]; is a type of amide binding [GO:0033218]; is a type of heterocyclic compound binding [GO:1901363]